cholesterol sulfotransferase activity [GO:0051922] (molecular function) References: PMID:11416019, PMID:12145317, PMID:12730293 Sources: RHEA:52368 Definition: Catalysis of the reaction: 3'-phosphoadenylyl sulfate + cholesterol = adenosine 3',5'-bisphosphate + cholesterol sulfate + H+. Relationships: is a type of alcohol sulfotransferase activity [GO:0004027]